{
  "term_label": "nucleus",
  "gene_name": "Transcription factor MafA",
  "gene": "UniProtKB:Q8NHW3",
  "gene_symbol": "MAFA",
  "term_id": "GO:0005634"
}